response to miconazole [GO:1905307] (biological process) Definition: Any process that results in a change in state or activity of a cell or an organism (in terms of movement, secretion, enzyme production, gene expression, etc.) as a result of a miconazole stimulus. Subtypes: cellular response to miconazole [GO:1905308] Relationships: is a type of response to nitrogen compound [GO:1901698] References: PMID:26108447 Sources: GOC:TermGenie, GO_REF:0000071